{
  "gene": "UniProtKB:Q8WWY7",
  "term_id": "GO:0004867",
  "gene_name": "WAP four-disulfide core domain protein 12",
  "gene_symbol": "WFDC12",
  "term_label": "serine-type endopeptidase inhibitor activity"
}